{
  "gene_name": "Cytochrome P450 2D6",
  "gene_symbol": "CYP2D6",
  "gene": "UniProtKB:P10635",
  "term_label": "oxidoreductase activity, acting on paired donors, with incorporation or reduction of molecular oxygen, reduced flavin or flavoprotein as one donor, and incorporation of one atom of oxygen",
  "term_id": "GO:0016712"
}